L-alanine transmembrane transport [GO:1904557] (biological process) Definition: The directed movement of L-alanine across a membrane by means of some agent such as a transporter or a pore. Subtypes: L-alanine export across the plasma membrane [GO:0140406], L-alanine import across plasma membrane [GO:1904273] Sources: GOC:TermGenie, GOC:kmv, GO_REF:0000069 Relationships: is a type of GO:0015808; is a type of L-alpha-amino acid transmembrane transport [GO:1902475]